{
  "gene_symbol": "SRPK3",
  "term_label": "regulation of mRNA processing",
  "term_id": "GO:0050684",
  "gene": "UniProtKB:Q9UPE1",
  "gene_name": "SRSF protein kinase 3"
}